regulation of leukocyte degranulation [GO:0043300] (biological process) Relationships: is a type of regulation of immune effector process [GO:0002697]; is a type of regulation of regulated secretory pathway [GO:1903305]; regulates leukocyte degranulation [GO:0043299] Also known as: regulation of immune cell degranulation, regulation of immune cell granule exocytosis, regulation of leucocyte degranulation, regulation of leukocyte granule exocytosis Subtypes: negative regulation of leukocyte degranulation [GO:0043301], GO:0043302, regulation of mast cell degranulation [GO:0043304], regulation of eosinophil degranulation [GO:0043309], GO:0043313, regulation of cytotoxic T cell degranulation [GO:0043317], GO:0043321, GO:1903581 Sources: GOC:add, ISBN:0781735149 Definition: Any process that modulates the frequency, rate, or extent of leukocyte degranulation.